{
  "term_id": "GO:0000977",
  "gene_name": "Zinc finger protein 529",
  "term_label": "RNA polymerase II transcription regulatory region sequence-specific DNA binding",
  "gene_symbol": "ZNF529",
  "gene": "UniProtKB:Q6P280"
}